{
  "gene_symbol": "HSD17B11",
  "gene_name": "Estradiol 17-beta-dehydrogenase 11",
  "term_id": "UNKNOWN:0002",
  "term_label": "Unknown biological process",
  "gene": "UniProtKB:Q8NBQ5"
}